ent-kaurenoic acid monooxygenase activity [GO:0051777] (molecular function) Also known as: ent-kaurenoate oxidase activity, ent-kaurenoic acid oxidase activity Definition: Catalysis of the reaction:ent-kaur-16-en-19-oate + 3 O2 + 3 reduced [NADPH--hemoprotein reductase] = gibberellin A12 + 4 H+ + 4 H2O + 3 oxidized [NADPH--hemoprotein reductase]. Catalyzes three successive oxidations of ent-kaurenoic acid. Sources: RHEA:33219 Relationships: is a type of oxidoreductase activity, acting on paired donors, with incorporation or reduction of molecular oxygen, reduced flavin or flavoprotein as one donor, and incorporation of one atom of oxygen [GO:0016712]